negative regulation of cell wall polysaccharide catabolic process [GO:2000967] (biological process) Also known as: negative regulation of cell wall polysaccharide breakdown Sources: GOC:mengo_curators Relationships: is_a GO:0009895; is_a negative regulation of macromolecule metabolic process [GO:0010605]; is_a negative regulation of carbohydrate metabolic process [GO:0045912]; is a type of regulation of cell wall polysaccharide catabolic process [GO:2000966]; negatively regulates cell wall polysaccharide catabolic process [GO:0044347] Definition: Any process that stops, prevents or reduces the frequency, rate or extent of cell wall polysaccharide catabolic process. Subtypes: negative regulation of plant-type cell wall cellulose catabolic process [GO:2000940], negative regulation of mannan catabolic process [GO:2000995]